{
  "term_id": "UNKNOWN:0003",
  "gene": "UniProtKB:A8MX19",
  "gene_name": "Putative protein FAM90A12P",
  "term_label": "Unknown cellular component",
  "gene_symbol": "FAM90A12P"
}